{
  "gene_symbol": "FGF9",
  "gene_name": "Fibroblast growth factor 9",
  "term_id": "GO:0008543",
  "gene": "UniProtKB:P31371",
  "term_label": "fibroblast growth factor receptor signaling pathway"
}